{
  "gene_name": "DNA damage-binding protein 1",
  "term_label": "site of double-strand break",
  "term_id": "GO:0035861",
  "gene_symbol": "DDB1",
  "gene": "UniProtKB:Q16531"
}